{
  "term_id": "GO:0001228",
  "gene_name": "Cyclic AMP-dependent transcription factor ATF-5",
  "term_label": "DNA-binding transcription activator activity, RNA polymerase II-specific",
  "gene_symbol": "ATF5",
  "gene": "UniProtKB:Q9Y2D1"
}